{
  "term_label": "histone deacetylase binding",
  "gene_symbol": "MIER1",
  "gene": "UniProtKB:Q8N108",
  "term_id": "GO:0042826",
  "gene_name": "Mesoderm induction early response protein 1"
}